internal N(7)-methylguanine-containing RNA reader activity [GO:0160089] (molecular function) Relationships: is a type of protein-RNA adaptor activity [GO:0140517]; has part RNA binding [GO:0003723] References: PMID:37379838 Definition: A protein adaptor that recognizes and binds an RNA molecule modified by N(7)-methylguanine (m7G), a modification present at internal sites of mRNAs and some non-coding RNAs.